{
  "gene": "UniProtKB:Q9NQX4",
  "term_label": "cytoplasm",
  "term_id": "GO:0005737",
  "gene_symbol": "MYO5C",
  "gene_name": "Unconventional myosin-Vc"
}